{
  "gene_symbol": "ADAMTSL2",
  "gene": "UniProtKB:Q86TH1",
  "term_id": "GO:0031012",
  "gene_name": "ADAMTS-like protein 2",
  "term_label": "extracellular matrix"
}